2,4-dienoyl-CoA reductase (NADPH) activity [GO:0008670] (molecular function) Sources: EC:1.3.1.34 Also known as: 4-enoyl coenzyme A (reduced nicotinamide adenine dinucleotide phosphate) reductase activity, 4-enoyl-CoA reductase (NADPH) activity, 4-enoyl-CoA reductase (NADPH2), 4-enoyl-CoA reductase activity, trans-2,3-didehydroacyl-CoA:NADP+ 4-oxidoreductase activity Relationships: is a type of oxidoreductase activity, acting on the CH-CH group of donors, NAD or NADP as acceptor [GO:0016628] Definition: Catalysis of the reactions: a 4,5-saturated-(2E)-enoyl-CoA + NADP+ = a (2E,4E)-dienoyl-CoA + H+ + NADPH, and a (2E,4Z)-dienoyl-CoA + H+ + NADPH = a 4,5-saturated-(2E)-enoyl-CoA + NADP+.